{
  "term_label": "neuron projection",
  "gene": "UniProtKB:Q92952",
  "gene_name": "Small conductance calcium-activated potassium channel protein 1",
  "gene_symbol": "KCNN1",
  "term_id": "GO:0043005"
}